{
  "gene": "UniProtKB:Q4ZHG4",
  "term_id": "UNKNOWN:0003",
  "gene_name": "Fibronectin type III domain-containing protein 1",
  "term_label": "Unknown cellular component",
  "gene_symbol": "FNDC1"
}